positive regulation of paraxial mesodermal cell fate determination [GO:0048346] (biological process) Definition: Any process that activates or increases the frequency, rate or extent of paraxial mesoderm cell fate determination. Sources: GOC:dgh Also known as: up regulation of paraxial mesodermal cell fate determination, up-regulation of paraxial mesodermal cell fate determination, upregulation of paraxial mesodermal cell fate determination, activation of paraxial mesodermal cell fate determination, stimulation of paraxial mesodermal cell fate determination Relationships: is a type of positive regulation of mesodermal cell fate determination [GO:0048336]; is a type of GO:0048345; positively regulates paraxial mesodermal cell fate determination [GO:0048344]